regulation of reciprocal meiotic recombination [GO:0010520] (biological process) Definition: Any process that modulates the frequency, rate or extent of recombination during meiosis. Reciprocal meiotic recombination is the cell cycle process in which double strand breaks are formed and repaired through a double Holliday junction intermediate. Relationships: is a type of regulation of DNA recombination [GO:0000018]; is a type of regulation of cell cycle process [GO:0010564]; is a type of regulation of reproductive process [GO:2000241]; RO_0002211 reciprocal meiotic recombination [GO:0007131] Subtypes: positive regulation of reciprocal meiotic recombination [GO:0010845], negative regulation of reciprocal meiotic recombination [GO:0045128] Sources: GOC:dph, GOC:tb